{
  "gene_name": "Ras-related protein Rab-5A",
  "term_id": "GO:0030139",
  "gene": "UniProtKB:P20339",
  "term_label": "endocytic vesicle",
  "gene_symbol": "RAB5A"
}